cytokine production involved in immune response [GO:0002367] (biological process) Definition: The appearance of a cytokine due to biosynthesis or secretion following a cellular stimulus contributing to an immune response, resulting in an increase in its intracellular or extracellular levels. Sources: GOC:add, GO_REF:0000022, ISBN:0781735149 Also known as: cytokine biosynthetic process involved in immune response, cytokine production during immune response, cytokine secretion during immune response, cytokine secretion involved in immune response Note: Note that this term is in the subset of terms that should not be used for direct gene product annotation. Instead, select one of the 'regulation' children terms. Relationships: is a type of cytokine production [GO:0001816]; is_a production of molecular mediator of immune response [GO:0002440]; BFO_0000050 immune response [GO:0006955] Subtypes: B cell cytokine production [GO:0002368], T cell cytokine production [GO:0002369], natural killer cell cytokine production [GO:0002370], GO:0002371, myeloid leukocyte cytokine production [GO:0061082] Regulation: regulated by regulation of cytokine production involved in immune response [GO:0002718]; negatively regulated by GO:0002719; positively regulated by positive regulation of cytokine production involved in immune response [GO:0002720]